PTB domain binding [GO:0051425] (molecular function) Also known as: PID binding, phosphotyrosine-interacting domain binding Definition: Binding to a phosphotyrosine-binding (PTB) Binding to a phosphotyrosine-bindin domain. References: PMID:15924411 Sources: Pfam:PF02174 Relationships: is a type of protein domain specific binding [GO:0019904]